{
  "gene": "UniProtKB:Q13112",
  "term_label": "nucleus",
  "gene_name": "Chromatin assembly factor 1 subunit B",
  "gene_symbol": "CHAF1B",
  "term_id": "GO:0005634"
}